locomotor rhythm [GO:0045475] (biological process) Relationships: is a type of locomotory behavior [GO:0007626]; is a type of GO:0048512 Also known as: circadian locomotor activity rhythm Regulation: regulated by regulation of locomotor rhythm [GO:1904059]; negatively regulated by negative regulation of locomotor rhythm [GO:1904060]; positively regulated by positive regulation of locomotor rhythm [GO:1904061] Sources: GOC:go_curators Definition: The rhythm of the locomotor activity of an organism during its 24 hour activity cycle.